{
  "gene_name": "Leucine-rich repeat-containing protein 4C",
  "term_label": "cell-cell adhesion mediator activity",
  "term_id": "GO:0098632",
  "gene": "UniProtKB:Q9HCJ2",
  "gene_symbol": "LRRC4C"
}